negative regulation of DNA endoreduplication [GO:0032876] (biological process) Definition: Any process that stops, prevents, or reduces the frequency, rate or extent of DNA endoreduplication. Sources: GOC:mah Also known as: down regulation of DNA endoreduplication, down-regulation of DNA endoreduplication, downregulation of DNA endoreduplication, negative regulation of DNA endoreplication, negative regulation of DNA re-duplication, inhibition of DNA endoreduplication Relationships: is a type of GO:0010948; is a type of GO:0032875; is a type of negative regulation of DNA-templated DNA replication [GO:2000104]; negatively regulates GO:0042023